{
  "gene": "UniProtKB:Q96FS4",
  "term_id": "UNKNOWN:0003",
  "gene_symbol": "SIPA1",
  "gene_name": "Signal-induced proliferation-associated protein 1",
  "term_label": "Unknown cellular component"
}